stalled ribosome sensor activity [GO:0170011] (MF) Definition: A molecule that recognizes stalled ribosomes and initiates a signaling response. Relationships: is a type of molecular sensor activity [GO:0140299]; has part ribosome binding [GO:0043022] References: PMID:32289254, PMID:32610081, PMID:36638793